regulation of pyocyanine biosynthetic process [GO:0062161] (BP) Also known as: regulation of pyocyanin biosynthetic process References: PMID:28715477 Subtypes: GO:0062162 Relationships: is a type of GO:0009889; regulates pyocyanine biosynthetic process [GO:0106220] Definition: Any process that modulates the frequency, rate or extent of a pyocyanine biosynthetic process.